detection of humidity [GO:0098513] (biological process) Sources: GOC:dos Definition: The series of events in which a humidity stimulus is received and converted into a molecular signal. Subtypes: detection of humidity stimulus involved in sensory perception [GO:0098512], detection of high humidity [GO:0098516], detection of low humidity [GO:0098517] Relationships: is_a detection of external stimulus [GO:0009581]; is a type of detection of abiotic stimulus [GO:0009582]